{
  "term_id": "GO:0005760",
  "gene": "UniProtKB:Q9UHN1",
  "gene_name": "DNA polymerase subunit gamma-2, mitochondrial",
  "term_label": "gamma DNA polymerase complex",
  "gene_symbol": "POLG2"
}